determination of digestive tract left/right asymmetry [GO:0071907] (biological process) Also known as: determination of gut left/right asymmetry, determination of left/right asymmetry of the digestive tract Subtypes: determination of intestine left/right asymmetry [GO:0071908], determination of stomach left/right asymmetry [GO:0071909] Definition: Determination of the asymmetric location of various parts of the digestive tract with respect to the left and right halves of the organism. The digestive tract is the anatomical structure through which food passes and is processed. Relationships: is a type of determination of left/right symmetry [GO:0007368]; is part of digestive tract development [GO:0048565] Sources: GOC:cvs